histone H3K23 acetyltransferase activity [GO:0043994] (molecular function) References: PMID:18552846, PMID:19056256 Note: Comment: Note that the residue position corresponds to the canonical human H3 histone (UniProtKB:P84243); this residue is conserved across all eukaryotes. Residue 1 is the first residue following removal of the initiating Methionine (Met). Note that each histone is encoded by multiple genes, and sequences may vary across different genes within an organism. Definition: Catalysis of the reaction: acetyl-CoA + histone H3 L-lysine (position 23) = CoA + histone H3 N6-acetyl-L-lysine (position 23). Also known as: histone H3-K23 acetyltransferase activity, histone acetylase activity (H3-K23 specific), histone acetyltransferase activity (H3-K23 specific), histone lysine N-acetyltransferase activity (H3-K23 specific) Relationships: is a type of histone H3 acetyltransferase activity [GO:0010484]